{
  "term_label": "extracellular matrix",
  "term_id": "GO:0031012",
  "gene_name": "Fibrinogen-like protein 1",
  "gene_symbol": "FGL1",
  "gene": "UniProtKB:Q08830"
}